intestinal lipid absorption [GO:0098856] (biological process) Relationships: is a type of intestinal absorption [GO:0050892] Regulation: regulated by regulation of intestinal lipid absorption [GO:1904729]; negatively regulated by negative regulation of intestinal lipid absorption [GO:1904730]; positively regulated by positive regulation of intestinal lipid absorption [GO:1904731] References: PMID:18768481 Sources: GOC:dos, GOC:sl Definition: A process in which lipids are taken up from the contents of the intestine. Subtypes: intestinal cholesterol absorption [GO:0030299], GO:0060752